detection of inactivity [GO:0014863] (biological process) Sources: GOC:mtg_muscle Subtypes: detection of muscle inactivity [GO:0014869] Relationships: is a type of response to inactivity [GO:0014854]; is a type of detection of stimulus [GO:0051606] Definition: The series of events in which a inactivity stimulus is received by a cell or organism and converted into a molecular signal.